{
  "gene_name": "Olfactory receptor 5K2",
  "term_id": "GO:0005549",
  "gene": "UniProtKB:Q8NHB8",
  "gene_symbol": "OR5K2",
  "term_label": "odorant binding"
}